{
  "gene_symbol": "LINC00518",
  "gene": "UniProtKB:Q8N0U6",
  "term_id": "UNKNOWN:0002",
  "gene_name": "Putative uncharacterized protein encoded by LINC00518",
  "term_label": "Unknown biological process"
}